plasmid partitioning [GO:0030541] (biological process) Sources: GOC:mah Relationships: is_a plasmid maintenance [GO:0006276] Subtypes: 2-micrometer plasmid partitioning [GO:0030543] Definition: Any process in which plasmids are segregated or distributed into daughter cells upon cell division.